{
  "term_label": "Unknown molecular function",
  "term_id": "UNKNOWN:0001",
  "gene": "UniProtKB:A0A0B4J262",
  "gene_symbol": "TRAV8-6",
  "gene_name": "T cell receptor alpha variable 8-6"
}